humoral immune response mediated by circulating immunoglobulin [GO:0002455] (biological process) Regulation: regulated by regulation of humoral immune response mediated by circulating immunoglobulin [GO:0002923]; negatively regulated by negative regulation of humoral immune response mediated by circulating immunoglobulin [GO:0002924]; positively regulated by GO:0002925 Relationships: is a type of humoral immune response [GO:0006959]; is a type of GO:0016064 Also known as: circulating antibody mediated immune response, circulating immunoglobulin mediated immune response, humoral immune response mediated by circulating antibody, humoral defence mechanism Definition: An immune response dependent upon secreted immunoglobulin. An example of this process is found in Mus musculus. Sources: GOC:add, GO_REF:0000022, ISBN:0781735149